 [go#goslim:flybase:ribbon] Note: Insecta GO ribbon slim